{
  "term_id": "GO:0046972",
  "gene_symbol": "KAT8",
  "term_label": "histone H4K16 acetyltransferase activity",
  "gene": "UniProtKB:Q9H7Z6",
  "gene_name": "Histone acetyltransferase KAT8"
}